selective angioblast sprouting [GO:0035474] (biological process) Definition: The segregation of angioblasts into discrete arterial and venous vessels from one common precursor vessel. References: PMID:19815777 Sources: GOC:dgh Relationships: is a type of anatomical structure formation involved in morphogenesis [GO:0048646]; is part of blood vessel morphogenesis [GO:0048514]